{
  "term_label": "cholesterol homeostasis",
  "gene": "UniProtKB:Q9UHC9",
  "gene_name": "NPC1-like intracellular cholesterol transporter 1",
  "term_id": "GO:0042632",
  "gene_symbol": "NPC1L1"
}